viral integration complex [GO:0019035] (cellular component) Also known as: PIC, pre-integration complex Relationships: is a type of protein-containing complex [GO:0032991]; is part of host cell [GO:0043657] References: PMID:21037296, PMID:2721960, PMID:29900498 Definition: A nucleoprotein complex containing viral genetic material and the viral integrase, required for genome integration into the host's genome. May contain other proteins.